{
  "gene_name": "Abscission_NoCut checkpoint regulator",
  "gene": "UniProtKB:Q96K21",
  "term_label": "mitotic cytokinesis checkpoint signaling",
  "gene_symbol": "ZFYVE19",
  "term_id": "GO:0044878"
}